{
  "gene_name": "Probable ribonuclease ZC3H12D",
  "gene_symbol": "ZC3H12D",
  "term_label": "3'-UTR-mediated mRNA destabilization",
  "gene": "UniProtKB:A2A288",
  "term_id": "GO:0061158"
}